{
  "gene_symbol": "NFXL1",
  "term_id": "GO:0005634",
  "term_label": "nucleus",
  "gene": "UniProtKB:Q6ZNB6",
  "gene_name": "NF-X1-type zinc finger protein NFXL1"
}